{
  "term_label": "Rho protein signal transduction",
  "gene_symbol": "RHOA",
  "gene_name": "Transforming protein RhoA",
  "term_id": "GO:0007266",
  "gene": "UniProtKB:P61586"
}